{
  "gene_symbol": "USP17L1",
  "gene_name": "Ubiquitin carboxyl-terminal hydrolase 17-like protein 1",
  "term_id": "GO:0042981",
  "term_label": "regulation of apoptotic process",
  "gene": "UniProtKB:Q7RTZ2"
}